{
  "term_id": "GO:0006081",
  "term_label": "aldehyde metabolic process",
  "gene_symbol": "ALDH3B1",
  "gene": "UniProtKB:P43353",
  "gene_name": "Aldehyde dehydrogenase family 3 member B1"
}